{
  "gene": "UniProtKB:Q9NYS0",
  "gene_symbol": "NKIRAS1",
  "term_label": "Unknown cellular component",
  "term_id": "UNKNOWN:0003",
  "gene_name": "NF-kappa-B inhibitor-interacting Ras-like protein 1"
}